protein localization to presynapse [GO:1905383] (BP) Regulation: RO_0002211 by regulation of protein localization to presynapse [GO:1905384]; negatively regulated by negative regulation of protein localization to presynapse [GO:1905385]; positively regulated by positive regulation of protein localization to presynapse [GO:1905386] Subtypes: anterograde axonal protein transport [GO:0099641], GO:0099644 Definition: A process in which a protein is transported to, or maintained in, a location within a presynapse. Also known as: protein localisation in presynapse, protein localisation to presynapse, protein localization in presynapse, recruitment of presynaptic proteins Relationships: is a type of protein localization to synapse [GO:0035418] References: PMID:24449494 Sources: GOC:TermGenie, GO_REF:0000087